{
  "gene": "UniProtKB:Q9P126",
  "term_label": "transmembrane signaling receptor activity",
  "gene_name": "C-type lectin domain family 1 member B",
  "term_id": "GO:0004888",
  "gene_symbol": "CLEC1B"
}